{
  "term_id": "GO:0004382",
  "gene_symbol": "ENTPD3",
  "term_label": "GDP phosphatase activity",
  "gene_name": "Ectonucleoside triphosphate diphosphohydrolase 3",
  "gene": "UniProtKB:O75355"
}